{
  "gene": "UniProtKB:Q96AQ2",
  "gene_name": "Transmembrane protein 125",
  "term_id": "UNKNOWN:0002",
  "gene_symbol": "TMEM125",
  "term_label": "Unknown biological process"
}